{
  "gene_symbol": "WNT3A",
  "term_label": "cytokine activity",
  "gene": "UniProtKB:P56704",
  "gene_name": "Protein Wnt-3a",
  "term_id": "GO:0005125"
}